amelogenesis [GO:0097186] (biological process) Definition: The process whose specific outcome is the formation of tooth enamel, occurring in two stages: secretory stage and maturation stage. Also known as: enamel development Relationships: is a type of GO:0042475; is a type of GO:0048646 References: PMID:10206335, PMID:21196346 Sources: GOC:cjm, GOC:sl